{
  "gene_symbol": "KISS1R",
  "term_label": "neuropeptide receptor activity",
  "gene": "UniProtKB:Q969F8",
  "term_id": "GO:0008188",
  "gene_name": "KiSS-1 receptor"
}